acid phosphatase activity [GO:0003993] (molecular function) Also known as: glycerophosphatase activity, phosphomonoesterase activity, acid monophosphatase activity, acid nucleoside diphosphate phosphatase activity, acid phosphohydrolase activity, acid phosphomonoester hydrolase activity, acid phosphomonoesterase activity, orthophosphoric-monoester phosphohydrolase (acid optimum), phosphate-monoester phosphohydrolase (acid optimum), uteroferrin Sources: EC:3.1.3.2 Relationships: is a type of GO:0016791 Definition: Catalysis of the reaction: an orthophosphoric monoester + H2O = an alcohol + phosphate, with an acid pH optimum.